{
  "term_id": "GO:0005737",
  "term_label": "cytoplasm",
  "gene_symbol": "PRUNE1",
  "gene_name": "Exopolyphosphatase PRUNE1",
  "gene": "UniProtKB:Q86TP1"
}